{
  "gene_symbol": "NSUN7",
  "gene": "UniProtKB:Q8NE18",
  "gene_name": "Putative methyltransferase NSUN7",
  "term_label": "Unknown cellular component",
  "term_id": "UNKNOWN:0003"
}